{
  "gene": "UniProtKB:Q658P3",
  "term_id": "GO:0015677",
  "gene_name": "Metalloreductase STEAP3",
  "term_label": "copper ion import",
  "gene_symbol": "STEAP3"
}